{
  "gene_symbol": "CNST",
  "gene_name": "Consortin",
  "gene": "UniProtKB:Q6PJW8",
  "term_id": "GO:0030133",
  "term_label": "transport vesicle"
}